phosphoprotein phosphatase activity [GO:0004721] (MF) Regulation: negatively regulated by protein phosphatase inhibitor activity [GO:0004864]; regulated by GO:0019888; positively regulated by GO:0072542 Also known as: phosphoprotein phosphohydrolase activity, protein phosphatase activity, protein phosphatase-1 activity, protein phosphatase-2A activity, protein phosphatase-2B activity, protein phosphatase-2C activity Definition: Catalysis of the reaction: a phosphoprotein + H2O = a protein + phosphate. Together with protein kinases, these enzymes control the state of phosphorylation of cellular proteins and thereby provide an important mechanism for regulating cellular activity. Subtypes: GO:0004722, protein tyrosine phosphatase activity [GO:0004725], protein tyrosine/serine/threonine phosphatase activity [GO:0008138], protein tyrosine/threonine phosphatase activity [GO:0008330], transmembrane receptor protein phosphatase activity [GO:0019198], MAP kinase phosphatase activity [GO:0033549], [hydroxymethylglutaryl-CoA reductase (NADPH)]-phosphatase activity [GO:0047384], [3-methyl-2-oxobutanoate dehydrogenase (lipoamide)]-phosphatase activity [GO:0047385], myosin-light-chain-phosphatase activity [GO:0050115], [phosphorylase] phosphatase activity [GO:0050196], [acetyl-CoA carboxylase]-phosphatase activity [GO:0050406], [glycogen-synthase-D] phosphatase activity [GO:0050407], GO:0050408, protein arginine phosphatase activity [GO:0098627], protein histidine phosphatase activity [GO:0101006], GO:0101014, GO:0140789 Relationships: is a type of phosphatase activity [GO:0016791]; is a type of GO:0140096 Sources: ISBN:0198547684